{
  "gene": "UniProtKB:Q6NSI4",
  "term_id": "GO:0005657",
  "term_label": "replication fork",
  "gene_symbol": "RADX",
  "gene_name": "RPA-related protein RADX"
}